epithelial tube branching involved in lung morphogenesis [GO:0060441] (biological process) Definition: The process in which a highly ordered sequence of patterning events generates the branched epithelial tubes of the lung, consisting of reiterated combinations of bud outgrowth, elongation, and dichotomous subdivision of terminal units. Sources: GOC:dph, GOC:mtg_lung Also known as: lung branching morphogenesis Subtypes: primary lung bud formation [GO:0060431] Regulation: regulated by regulation of branching involved in lung morphogenesis [GO:0061046]; positively regulated by positive regulation of branching involved in lung morphogenesis [GO:0061047]; negatively regulated by negative regulation of branching involved in lung morphogenesis [GO:0061048] Relationships: is a type of GO:0048754; is part of lung morphogenesis [GO:0060425]